{
  "gene_name": "S-arrestin",
  "term_label": "photoreceptor outer segment",
  "gene": "UniProtKB:P10523",
  "gene_symbol": "SAG",
  "term_id": "GO:0001750"
}